{
  "gene_name": "Diphthamide biosynthesis protein 3",
  "term_label": "protein histidyl modification to diphthamide",
  "gene": "UniProtKB:Q96FX2",
  "gene_symbol": "DPH3",
  "term_id": "GO:0017183"
}